{
  "term_id": "UNKNOWN:0002",
  "gene": "UniProtKB:Q8IV35",
  "gene_name": "WD repeat-containing protein 49",
  "gene_symbol": "WDR49",
  "term_label": "Unknown biological process"
}